snRNA metabolic process [GO:0016073] (biological process) Subtypes: snRNA transcription [GO:0009301], snRNA catabolic process [GO:0016076], snRNA processing [GO:0016180] Definition: The chemical reactions and pathways involving snRNA, small nuclear RNA, any of various low-molecular-mass RNA molecules found in the eukaryotic nucleus as components of the small nuclear ribonucleoprotein. Sources: ISBN:0198506732 Also known as: snRNA metabolism Relationships: is a type of RNA metabolic process [GO:0016070]